{
  "gene": "UniProtKB:A0A7P0TAN4",
  "term_id": "GO:0001228",
  "gene_name": "Uncharacterized protein",
  "gene_symbol": "LOC122539214",
  "term_label": "DNA-binding transcription activator activity, RNA polymerase II-specific"
}